{
  "gene": "UniProtKB:P10599",
  "gene_name": "Thioredoxin",
  "gene_symbol": "TXN",
  "term_label": "Unknown cellular component",
  "term_id": "UNKNOWN:0003"
}